{
  "term_label": "cholesterol binding",
  "gene": "UniProtKB:Q969R2",
  "term_id": "GO:0015485",
  "gene_symbol": "OSBP2",
  "gene_name": "Oxysterol-binding protein 2"
}